{
  "gene": "UniProtKB:P51690",
  "gene_symbol": "ARSL",
  "term_label": "Unknown biological process",
  "gene_name": "Arylsulfatase L",
  "term_id": "UNKNOWN:0002"
}